{
  "term_id": "GO:0038062",
  "gene": "UniProtKB:Q08345",
  "term_label": "protein tyrosine kinase collagen receptor activity",
  "gene_symbol": "DDR1",
  "gene_name": "Epithelial discoidin domain-containing receptor 1"
}